histone H4S1 kinase activity [GO:0044023] (molecular function) Also known as: histone kinase activity (H4-S1 specific), histone serine kinase activity (H4-S1 specific), histone-serine kinase activity (H4-S1 specific) Sources: GOC:jl Relationships: is a type of protein serine/threonine kinase activity [GO:0004674]; is a type of histone H4 kinase activity [GO:0140997] Definition: Catalysis of the reaction: histone H4-serine (position 1) + ATP = histone H4-phosphoserine (position 1) + ADP. This reaction is the addition of a phosphate group to the serine residue at position 1 of histone H4. Note: Note that the residue position corresponds to the canonical human H4 histone (UniProtKB:P02309); this residue is conserved across all eukaryotes, but is a Thr in Drosophila. Note that the initiation methionine is cleaved, so the first residue is S1.